{
  "term_id": "GO:0050830",
  "gene_name": "Guanylate-binding protein 2",
  "term_label": "defense response to Gram-positive bacterium",
  "gene_symbol": "GBP2",
  "gene": "UniProtKB:P32456"
}